{
  "term_id": "UNKNOWN:0002",
  "gene_name": "MOB-like protein phocein",
  "gene": "UniProtKB:Q9Y3A3",
  "gene_symbol": "MOB4",
  "term_label": "Unknown biological process"
}